ubiquinone biosynthetic process [GO:0006744] (BP) Definition: The chemical reactions and pathways resulting in the formation of ubiquinone, a lipid-soluble electron-transporting coenzyme. Sources: GOC:mah Relationships: is a type of ubiquinone metabolic process [GO:0006743]; is_a GO:1901663 Also known as: coenzyme Q biosynthesis, coenzyme Q biosynthetic process, ubiquinone anabolism, ubiquinone biosynthesis, ubiquinone formation, ubiquinone synthesis, coenzyme Q10 biosynthesis, coenzyme Q10 biosynthetic process, coenzyme Q6 biosynthesis, coenzyme Q6 biosynthetic process, coenzyme Q8 biosynthesis, coenzyme Q8 biosynthetic process, coenzyme Q9 biosynthesis, coenzyme Q9 biosynthetic process Regulation: RO_0002211 by regulation of ubiquinone biosynthetic process [GO:0010795]; negatively regulated by negative regulation of ubiquinone biosynthetic process [GO:1904774]; positively regulated by positive regulation of ubiquinone biosynthetic process [GO:1904775]